{
  "gene_symbol": "BMPR1B",
  "term_id": "GO:0043235",
  "gene_name": "Bone morphogenetic protein receptor type-1B",
  "gene": "UniProtKB:O00238",
  "term_label": "receptor complex"
}